rhabdomere microvillus membrane [GO:0035997] (cellular component) References: PMID:14744998 Sources: GOC:bf, GOC:sart Definition: The portion of the plasma membrane surrounding a microvillus of a rhabdomere. Relationships: is_a microvillus membrane [GO:0031528]; is part of rhabdomere membrane [GO:0033583]; is part of rhabdomere microvillus [GO:0035996]